reactive nitrogen species metabolic process [GO:2001057] (biological process) Subtypes: GO:0042126, GO:0046209 Relationships: is a type of metabolic process [GO:0008152] Sources: GOC:obol Definition: The chemical reactions and pathways involving a reactive nitrogen species. Also known as: RNS metabolic process, RNS metabolism, reactive nitrogen species metabolism